{
  "gene_name": "Small integral membrane protein 3",
  "term_id": "UNKNOWN:0002",
  "gene_symbol": "SMIM3",
  "term_label": "Unknown biological process",
  "gene": "UniProtKB:Q9BZL3"
}